negative regulation of synaptic vesicle transport [GO:1902804] (biological process) References: PMID:23527112 Sources: GOC:TermGenie, GOC:kmv, GO_REF:0000058 Also known as: down regulation of synaptic vesicle transport, down-regulation of synaptic vesicle transport, downregulation of synaptic vesicle transport, inhibition of synaptic vesicle transport, down regulation of synaptic vesicle fission, down regulation of synaptic vesicle fusion, down-regulation of synaptic vesicle fission, down-regulation of synaptic vesicle fusion, downregulation of synaptic vesicle fission, downregulation of synaptic vesicle fusion, inhibition of synaptic vesicle fission, inhibition of synaptic vesicle fusion, negative regulation of synaptic vesicle fission, negative regulation of synaptic vesicle fusion Definition: Any process that stops, prevents or reduces the frequency, rate or extent of synaptic vesicle transport. Subtypes: GO:1903743 Relationships: is a type of negative regulation of cellular process [GO:0048523]; is a type of negative regulation of transport [GO:0051051]; is a type of regulation of synaptic vesicle transport [GO:1902803]; negatively regulates synaptic vesicle transport [GO:0048489]